{
  "gene_symbol": "KCNS2",
  "gene": "UniProtKB:Q9ULS6",
  "term_label": "potassium channel regulator activity",
  "term_id": "GO:0015459",
  "gene_name": "Potassium voltage-gated channel subfamily S member 2"
}